{
  "term_label": "detection of calcium ion",
  "gene_symbol": "CALM3",
  "gene": "UniProtKB:P0DP25",
  "gene_name": "Calmodulin-3",
  "term_id": "GO:0005513"
}